{
  "gene_name": "Coatomer subunit beta",
  "gene": "UniProtKB:P53618",
  "term_label": "endoplasmic reticulum to Golgi vesicle-mediated transport",
  "term_id": "GO:0006888",
  "gene_symbol": "COPB1"
}